{
  "term_label": "dynein intermediate chain binding",
  "gene_name": "Dynein axonemal heavy chain 7",
  "term_id": "GO:0045505",
  "gene": "UniProtKB:Q8WXX0",
  "gene_symbol": "DNAH7"
}